{
  "term_label": "mitochondrion",
  "gene_symbol": "SLC25A53",
  "gene": "UniProtKB:Q5H9E4",
  "term_id": "GO:0005739",
  "gene_name": "Solute carrier family 25 member 53"
}